{
  "term_id": "GO:0005615",
  "gene_name": "Insulin-like growth factor-binding protein 7",
  "term_label": "extracellular space",
  "gene": "UniProtKB:Q16270",
  "gene_symbol": "IGFBP7"
}